energy taxis [GO:0009453] (biological process) Also known as: energytaxis, taxis in response to energy source Relationships: is a type of taxis [GO:0042330] References: PMID:11029423 Sources: GOC:jl Definition: The directed movement of a motile cell or organism in response to physical parameters involved in energy generation, such as light, oxygen, and oxidizable substrates. Subtypes: aerotaxis [GO:0009454], GO:0009455, phototaxis [GO:0042331], chemotaxis to oxidizable substrate [GO:0042333], taxis to electron acceptor [GO:0042334], positive energy taxis [GO:0052128], negative energy taxis [GO:0052129]